{
  "gene_name": "Putative ferritin heavy polypeptide-like 19",
  "gene_symbol": "FTH1P19",
  "gene": "UniProtKB:P0C7X4",
  "term_id": "UNKNOWN:0002",
  "term_label": "Unknown biological process"
}